{
  "term_id": "GO:0005770",
  "gene_symbol": "VPS41",
  "gene": "UniProtKB:P49754",
  "gene_name": "Vacuolar protein sorting-associated protein 41 homolog",
  "term_label": "late endosome"
}